(R)-mandelate dehydrogenase activity [GO:0097620] (molecular function) Relationships: is a type of oxidoreductase activity, acting on CH-OH group of donors [GO:0016614] Definition: Catalysis of the reaction: (R)-2-hydroxy-2-phenylacetate + acceptor = phenylglyoxylate + reduced acceptor. Note: In the yeast Rhodotorula graminis, (R)-mandelate dehydrogenase is the first enzyme of the mandelate pathway, and catalyzes the NAD-dependent oxidation of (R)-mandelate to phenylglyoxylate. Also known as: D-mandelate dehydrogenase activity References: PMID:1731758 Sources: GOC:pr, RHEA:43112